{
  "gene_symbol": "COL11A1",
  "gene": "UniProtKB:P12107",
  "term_id": "GO:0030020",
  "gene_name": "Collagen alpha-1(XI) chain",
  "term_label": "extracellular matrix structural constituent conferring tensile strength"
}